{
  "gene_name": "Zinc finger protein 479",
  "gene": "UniProtKB:Q96JC4",
  "term_id": "GO:0000978",
  "term_label": "RNA polymerase II cis-regulatory region sequence-specific DNA binding",
  "gene_symbol": "ZNF479"
}